mannoside alpha-1,4-mannosidase activity [GO:0052766] (molecular function) Definition: Catalysis of the hydrolysis of the alpha-(1->4) linkage of the terminal, non-reducing alpha-D-mannose residues in alpha-D-mannosides. References: PMID:20081828 Sources: GOC:mengo_curators Also known as: alpha-1,4-exomannosidase activity, alpha-1,4-mannosidase activity, mannoside alpha-1,4-exomannosidase activity, mannoside exo-alpha-1,4-mannosidase activity Relationships: is a type of alpha-mannosidase activity [GO:0004559]